{
  "term_label": "plasma membrane",
  "gene_name": "Unconventional myosin-VI",
  "gene_symbol": "MYO6",
  "term_id": "GO:0005886",
  "gene": "UniProtKB:Q9UM54"
}